{
  "term_id": "GO:0030154",
  "term_label": "cell differentiation",
  "gene_symbol": "NKX3-1",
  "gene": "UniProtKB:Q99801",
  "gene_name": "Homeobox protein Nkx-3.1"
}